establishment of mitotic spindle localization [GO:0040001] (biological process) Definition: The cell cycle process in which the directed movement of the mitotic spindle to a specific location in the cell occurs. Subtypes: establishment of mitotic spindle orientation [GO:0000132] Regulation: regulated by Wnt signaling pathway, regulating spindle positioning [GO:0060069] Sources: GOC:ai Relationships: is a type of establishment of spindle localization [GO:0051293]; is_a microtubule cytoskeleton organization involved in mitosis [GO:1902850] Also known as: establishment of mitotic spindle localisation, mitotic spindle positioning, mitotic spindle positioning or orientation, spindle positioning involved in mitotic cell cycle, mitotic spindle positioning and orientation, spindle positioning during mitosis